{
  "term_label": "Unknown biological process",
  "gene_symbol": "LBHD2",
  "term_id": "UNKNOWN:0002",
  "gene_name": "LBH domain-containing protein 2",
  "gene": "UniProtKB:A0A0U1RRK4"
}